regulation of potassium ion transport [GO:0043266] (biological process) Sources: GOC:jl Also known as: regulation of K+ transport, regulation of potassium transport, regulation of K+ conductance, regulation of potassium conductance, regulation of potassium ion conductance Definition: Any process that modulates the frequency, rate or extent of the directed movement of potassium ions (K+) into, out of or within a cell, or between cells, by means of some agent such as a transporter or pore. Relationships: is a type of GO:0010959; regulates potassium ion transport [GO:0006813] Subtypes: negative regulation of potassium ion transport [GO:0043267], positive regulation of potassium ion transport [GO:0043268], regulation of potassium ion transmembrane transport [GO:1901379]